{
  "gene": "UniProtKB:Q96PX9",
  "gene_name": "Pleckstrin homology domain-containing family G member 4B",
  "term_label": "guanyl-nucleotide exchange factor activity",
  "gene_symbol": "PLEKHG4B",
  "term_id": "GO:0005085"
}